{
  "term_label": "nuclear polyadenylation-dependent CUT catabolic process",
  "gene_symbol": "EXOSC10",
  "gene": "UniProtKB:Q01780",
  "gene_name": "Exosome component 10",
  "term_id": "GO:0071039"
}